{
  "term_label": "myosin filament",
  "gene_symbol": "MYH11",
  "gene": "UniProtKB:P35749",
  "gene_name": "Myosin-11",
  "term_id": "GO:0032982"
}